{
  "gene": "UniProtKB:Q8IZP0",
  "term_label": "lamellipodium",
  "gene_symbol": "ABI1",
  "gene_name": "Abl interactor 1",
  "term_id": "GO:0030027"
}